{
  "term_label": "olfactory receptor activity",
  "gene": "UniProtKB:Q8NGA1",
  "gene_name": "Olfactory receptor 1M1",
  "term_id": "GO:0004984",
  "gene_symbol": "OR1M1"
}